{
  "gene": "UniProtKB:Q9BRI3",
  "term_id": "GO:0071577",
  "gene_symbol": "SLC30A2",
  "gene_name": "Proton-coupled zinc antiporter SLC30A2",
  "term_label": "zinc ion transmembrane transport"
}